{
  "term_id": "UNKNOWN:0003",
  "term_label": "Unknown cellular component",
  "gene_symbol": "MUC15",
  "gene": "UniProtKB:Q8N387",
  "gene_name": "Mucin-15"
}